{
  "term_id": "GO:0003700",
  "gene_symbol": "GTF2IRD1",
  "gene_name": "General transcription factor II-I repeat domain-containing protein 1",
  "term_label": "DNA-binding transcription factor activity",
  "gene": "UniProtKB:Q9UHL9"
}